positive regulation of amide catabolic process [GO:0034253] (BP) Also known as: positive regulation of amide breakdown, positive regulation of amide catabolism, positive regulation of cellular amide catabolic process, positive regulation of amide degradation Sources: GOC:mah Relationships: is a type of GO:0009896; is a type of positive regulation of amide metabolic process [GO:0034250]; is a type of GO:0034251; positively regulates GO:0043605 Subtypes: GO:1901714 Definition: Any process that activates or increases the frequency, rate or extent of the chemical reactions and pathways resulting in the breakdown of amides.